{
  "gene_name": "Disintegrin and metalloproteinase domain-containing protein 8",
  "gene_symbol": "ADAM8",
  "term_id": "GO:0050839",
  "gene": "UniProtKB:P78325",
  "term_label": "cell adhesion molecule binding"
}